negative regulation of translational initiation in response to starvation [GO:0071263] (biological process) Also known as: down regulation of translation initiation in response to starvation, down-regulation of translation initiation in response to starvation, downregulation of translation initiation in response to starvation, negative regulation of translational initiation in response to nutrient starvation, inhibition of translation initiation in response to starvation Definition: Any process that stops, prevents or reduces the rate of translation initiation, as a result of deprivation of nourishment. Sources: GOC:mah Relationships: is a type of negative regulation of translation in response to stress [GO:0032055]; is a type of negative regulation of translational initiation in response to stress [GO:0032057]; is_a regulation of translational initiation in response to starvation [GO:0071262]